{
  "gene_name": "F-box only protein 44",
  "gene": "UniProtKB:Q9H4M3",
  "term_label": "SCF ubiquitin ligase complex",
  "term_id": "GO:0019005",
  "gene_symbol": "FBXO44"
}